primary fluorescent dioxobilin-type chlorophyll catabolite methylesterase activity [GO:0106372] (molecular function) Definition: Catalysis of the reaction: H2O + primary fluorescent dioxobilin-type chlorophyll catabolite = H+ + methanol + O13(4)-desmethyl pFCC. References: PMID:23723324 Sources: RHEA:67176 Relationships: is a type of carboxylic ester hydrolase activity [GO:0052689]